{
  "gene": "UniProtKB:Q01523",
  "gene_symbol": "DEFA5",
  "term_label": "antimicrobial humoral immune response mediated by antimicrobial peptide",
  "term_id": "GO:0061844",
  "gene_name": "Defensin alpha 5"
}